{
  "gene_name": "Semaphorin-3A",
  "term_label": "glutamatergic synapse",
  "term_id": "GO:0098978",
  "gene": "UniProtKB:Q14563",
  "gene_symbol": "SEMA3A"
}